interleukin-27 binding [GO:0045513] (molecular function) Relationships: is a type of interleukin-17 binding [GO:0019975] Definition: Binding to interleukin-27. Also known as: IL-27 binding Sources: GOC:go_curators